DnaB-DnaC-DnaT-PriA-PriC complex [GO:1990159] (cellular component) Relationships: is a type of pre-primosome complex [GO:1990099]; has part DnaB-DnaC complex [GO:1990100] References: PMID:8663105 Sources: GOC:bhm Also known as: DnaB-DnaC-DnaT-PriA-PriC preprimosome, phi-X174-type preprimosome Definition: A protein-DNA complex consisting of the helicase loading complex DnaB-DnaC, replication restart proteins DnaT, PriA and PriC, and associated DNA. Involved in the restart of DNA replication after a stalled replication fork has been repaired.